{
  "gene": "UniProtKB:Q9NUQ9",
  "term_id": "GO:0050870",
  "gene_name": "CYFIP-related Rac1 interactor B",
  "gene_symbol": "CYRIB",
  "term_label": "positive regulation of T cell activation"
}